{
  "gene_name": "CLIP-associating protein 1",
  "gene": "UniProtKB:Q7Z460",
  "term_label": "cytoplasmic microtubule",
  "term_id": "GO:0005881",
  "gene_symbol": "CLASP1"
}